{
  "gene": "UniProtKB:Q8TB72",
  "gene_symbol": "PUM2",
  "term_id": "GO:0043488",
  "gene_name": "Pumilio homolog 2",
  "term_label": "regulation of mRNA stability"
}